{
  "gene_name": "Signal-induced proliferation-associated 1-like protein 2",
  "term_label": "GTPase activator activity",
  "term_id": "GO:0005096",
  "gene_symbol": "SIPA1L2",
  "gene": "UniProtKB:Q9P2F8"
}